{
  "term_id": "GO:0031731",
  "gene_symbol": "DEFB130B",
  "gene": "UniProtKB:P0DP73",
  "gene_name": "Beta-defensin 130B",
  "term_label": "CCR6 chemokine receptor binding"
}